lipoate transmembrane transport [GO:0170006] (biological process) Definition: The process in which lipoate is transported across a membrane. References: PMID:20980265, PMID:25971966 Relationships: is a type of transmembrane transport [GO:0055085]